negative regulation of transcription by competitive promoter binding [GO:0010944] (biological process) Definition: Any process that stops, prevents, or reduces the frequency, rate or extent of DNA-dependent transcription using a mechanism that involves direct competition for interaction with a promoter binding site. Sources: GOC:tb Relationships: is a type of negative regulation of DNA-templated transcription [GO:0045892]